phospholipase C activator activity [GO:0160185] (molecular function) References: PMID:28130414 Definition: Binds to and increases the activity of the enzyme phospholipase C. Relationships: is a type of phospholipase activator activity [GO:0016004]; positively regulates phospholipase C activity [GO:0004629]